respiratory burst involved in defense response [GO:0002679] (biological process) Definition: A phase of elevated metabolic activity, during which oxygen consumption increases made as part of a defense response ; this leads to the production, by an NADH dependent system, of hydrogen peroxide (H2O2), superoxide anions and hydroxyl radicals. Relationships: is a type of immune effector process [GO:0002252]; is a type of respiratory burst [GO:0045730]; is part of defense response [GO:0006952] Subtypes: respiratory burst involved in inflammatory response [GO:0002536], respiratory burst after phagocytosis [GO:0045728] References: PMID:12789499 Sources: GOC:add, ISBN:0781735149